{
  "gene_symbol": "GSTP1",
  "gene": "UniProtKB:P09211",
  "term_id": "GO:0004364",
  "gene_name": "Glutathione S-transferase P",
  "term_label": "glutathione transferase activity"
}